{
  "term_id": "UNKNOWN:0003",
  "gene_name": "Protein FAM118B",
  "term_label": "Unknown cellular component",
  "gene_symbol": "FAM118B",
  "gene": "UniProtKB:Q9BPY3"
}